{
  "gene": "UniProtKB:Q86Y33",
  "term_label": "anaphase-promoting complex binding",
  "gene_name": "Cell division cycle protein 20 homolog B",
  "term_id": "GO:0010997",
  "gene_symbol": "CDC20B"
}